{
  "gene": "UniProtKB:Q9P1P4",
  "term_id": "GO:0001594",
  "term_label": "trace-amine receptor activity",
  "gene_name": "Putative trace amine-associated receptor 3",
  "gene_symbol": "TAAR3P"
}